{
  "gene_symbol": "PROK1",
  "term_label": "endothelial cell proliferation",
  "term_id": "GO:0001935",
  "gene_name": "Prokineticin-1",
  "gene": "UniProtKB:P58294"
}